colicin transport [GO:0042914] (biological process) Subtypes: group A colicin transport [GO:0042915] References: PMID:17347522 Sources: GOC:jl Relationships: is a type of bacteriocin transport [GO:0043213] Definition: The directed movement of a colicin into, out of or within a cell, or between cells, by means of some agent such as a transporter or pore. Colicins are a group of antibiotics produced by E. coli and related species that are encoded by a group of naturally occurring plasmids, e.g. Col E1.